{
  "gene_symbol": "FSCN1",
  "term_label": "actin filament bundle assembly",
  "gene_name": "Fascin",
  "term_id": "GO:0051017",
  "gene": "UniProtKB:Q16658"
}